{
  "gene": "UniProtKB:O43566",
  "gene_symbol": "RGS14",
  "term_label": "cytoplasm",
  "term_id": "GO:0005737",
  "gene_name": "Regulator of G-protein signaling 14"
}